{
  "gene_name": "PDZ domain-containing protein 9",
  "term_id": "UNKNOWN:0002",
  "gene_symbol": "PDZD9",
  "gene": "UniProtKB:Q8IXQ8",
  "term_label": "Unknown biological process"
}